{
  "gene": "UniProtKB:G3V523",
  "gene_symbol": "LOC730098",
  "term_id": "UNKNOWN:0002",
  "gene_name": "HCG2040265, isoform CRA_a",
  "term_label": "Unknown biological process"
}